{
  "gene_name": "MyoD family inhibitor",
  "term_label": "regulation of Wnt signaling pathway",
  "gene": "UniProtKB:Q99750",
  "gene_symbol": "MDFI",
  "term_id": "GO:0030111"
}